{
  "gene_name": "Protein Hook homolog 2",
  "gene_symbol": "HOOK2",
  "gene": "UniProtKB:Q96ED9",
  "term_label": "cytoskeleton-dependent intracellular transport",
  "term_id": "GO:0030705"
}